{
  "gene": "UniProtKB:P63128",
  "gene_name": "Endogenous retrovirus group K member 9 Pol protein",
  "gene_symbol": "ERVK-9",
  "term_label": "Unknown cellular component",
  "term_id": "UNKNOWN:0003"
}